{
  "gene": "UniProtKB:P42338",
  "term_id": "GO:0016477",
  "term_label": "cell migration",
  "gene_name": "Phosphatidylinositol 4,5-bisphosphate 3-kinase catalytic subunit beta isoform",
  "gene_symbol": "PIK3CB"
}